{
  "term_id": "GO:0000785",
  "gene": "UniProtKB:Q8WUB8",
  "gene_name": "PHD finger protein 10",
  "term_label": "chromatin",
  "gene_symbol": "PHF10"
}